{
  "gene_name": "Hypoxia-inducible factor 3-alpha",
  "gene": "UniProtKB:Q9Y2N7",
  "term_id": "GO:0000981",
  "gene_symbol": "HIF3A",
  "term_label": "DNA-binding transcription factor activity, RNA polymerase II-specific"
}